{
  "term_label": "structural constituent of skin epidermis",
  "gene_symbol": "KRT24",
  "term_id": "GO:0030280",
  "gene": "UniProtKB:Q2M2I5",
  "gene_name": "Keratin, type I cytoskeletal 24"
}